{
  "term_id": "GO:0003924",
  "term_label": "GTPase activity",
  "gene_name": "Guanine nucleotide-binding protein G(i) subunit alpha-2",
  "gene_symbol": "GNAI2",
  "gene": "UniProtKB:P04899"
}